{
  "gene_name": "Immunoglobulin heavy variable 3-30-5",
  "gene_symbol": "IGHV3-30-5",
  "term_label": "immunoglobulin mediated immune response",
  "gene": "UniProtKB:P0DP03",
  "term_id": "GO:0016064"
}